{
  "gene": "UniProtKB:O75952",
  "gene_name": "Calcium-binding tyrosine phosphorylation-regulated protein",
  "gene_symbol": "CABYR",
  "term_id": "UNKNOWN:0002",
  "term_label": "Unknown biological process"
}